axonemal B tubule inner sheath [GO:0160112] (CC) Definition: A structural network of microtubule inner proteins (MIPs) located inside the lumen of the B tubule of the axonemal microtubule doublet that helps stabilize the B tubule. Relationships: is a type of GO:0110165; is part of A axonemal microtubule [GO:0097649]; is part of axonemal microtubule doublet inner sheath [GO:0160110] References: PMID:29430673, PMID:37295417 Sources: GOC:krc